TMP metabolic process [GO:0046044] (biological process) Also known as: TMP metabolism Sources: GOC:go_curators Relationships: is a type of pyrimidine ribonucleoside monophosphate metabolic process [GO:0009173]; is_a pyrimidine ribonucleotide metabolic process [GO:0009218] Subtypes: TMP biosynthetic process [GO:0006230], TMP catabolic process [GO:0046045] Definition: The chemical reactions and pathways involving TMP, ribosylthymine monophosphate.